positive regulation of oligopeptide transport [GO:2000878] (biological process) Sources: GOC:obol Definition: Any process that activates or increases the frequency, rate or extent of oligopeptide transport. Relationships: is a type of positive regulation of transport [GO:0051050]; is a type of regulation of oligopeptide transport [GO:0090088]; positively regulates oligopeptide transport [GO:0006857] Subtypes: positive regulation of dipeptide transport [GO:2000880]